{
  "gene": "UniProtKB:Q8IWV2",
  "gene_symbol": "CNTN4",
  "term_id": "GO:0030424",
  "term_label": "axon",
  "gene_name": "Contactin-4"
}